{
  "term_id": "GO:0071805",
  "gene_name": "Potassium voltage-gated channel subfamily H member 3",
  "gene_symbol": "KCNH3",
  "gene": "UniProtKB:Q9ULD8",
  "term_label": "potassium ion transmembrane transport"
}